{
  "gene_name": "GRB2-related adapter protein 2",
  "term_label": "plasma membrane",
  "term_id": "GO:0005886",
  "gene_symbol": "GRAP2",
  "gene": "UniProtKB:O75791"
}